{
  "term_label": "Unknown biological process",
  "term_id": "UNKNOWN:0002",
  "gene": "UniProtKB:Q6GMR7",
  "gene_symbol": "FAAH2",
  "gene_name": "Fatty-acid amide hydrolase 2"
}